{
  "term_id": "GO:0005737",
  "term_label": "cytoplasm",
  "gene_name": "Cyclin-dependent kinase 15",
  "gene": "UniProtKB:Q96Q40",
  "gene_symbol": "CDK15"
}